{
  "term_label": "actin filament binding",
  "term_id": "GO:0051015",
  "gene_name": "GAS2-like protein 2",
  "gene": "UniProtKB:Q8NHY3",
  "gene_symbol": "GAS2L2"
}